ACP-dependent peptidyl-lysine N6-palmitoyltransferase activity [GO:0140771] (molecular function) References: PMID:32461253 Sources: RHEA:70615 Definition: Catalysis of the reaction: hexadecanoyl-[ACP] + L-lysyl-[protein] = H+ + holo-[ACP] + N(6)-hexadecanoyl-L-lysyl-[protein]. Relationships: is a type of GO:0018031